{
  "gene": "UniProtKB:Q15424",
  "gene_name": "Scaffold attachment factor B1",
  "gene_symbol": "SAFB",
  "term_id": "GO:0005634",
  "term_label": "nucleus"
}